tRNA-guanosine(34) queuine transglycosylase activity [GO:0008479] (molecular function) Also known as: Q-insertase, TGT, queuine tRNA-ribosyltransferase activity, tRNA guanine transglycosylase, tRNA transglycosylase, eTGT, queuine tRNA-ribosyltransferase, queuine(34) transfer ribonucleate ribosyltransferase, tRNA-guanosine(34) queuine transglycosylase, guanine insertion enzyme Relationships: is a type of pentosyltransferase activity [GO:0016763]; is a type of GO:0140101 Sources: RHEA:16633 Definition: Catalysis of the reaction: guanosine34 in tRNA + queuine = guanine + queuosine34 in tRNA.